{
  "term_label": "Unknown molecular function",
  "term_id": "UNKNOWN:0001",
  "gene_name": "piRNA biogenesis protein EXD1",
  "gene_symbol": "EXD1",
  "gene": "UniProtKB:Q8NHP7"
}